{
  "gene_name": "Probable cytosolic iron-sulfur protein assembly protein CIAO1",
  "term_id": "GO:0016226",
  "gene_symbol": "CIAO1",
  "term_label": "iron-sulfur cluster assembly",
  "gene": "UniProtKB:O76071"
}